regulation of protein neddylation [GO:2000434] (biological process) Relationships: is a type of regulation of protein modification by small protein conjugation or removal [GO:1903320]; regulates GO:0045116 Definition: Any process that modulates the frequency, rate or extent of protein neddylation. Also known as: regulation of RUB1-protein conjugation Sources: GOC:obol Subtypes: GO:2000435, positive regulation of protein neddylation [GO:2000436]